xanthosine transmembrane transporter activity [GO:0015553] (molecular function) Sources: ISBN:0198506732 Relationships: is a type of GO:0015211; is part of GO:0015863 Subtypes: GO:0015537 Definition: Enables the transfer of xanthosine, xanthine riboside, from one side of a membrane to the other.